{
  "term_label": "cell surface receptor protein tyrosine kinase signaling pathway",
  "gene_symbol": "DDR1",
  "gene_name": "Epithelial discoidin domain-containing receptor 1",
  "gene": "UniProtKB:Q08345",
  "term_id": "GO:0007169"
}